{
  "term_id": "GO:0001916",
  "term_label": "positive regulation of T cell mediated cytotoxicity",
  "gene_symbol": "ULBP1",
  "gene": "UniProtKB:Q9BZM6",
  "gene_name": "UL16-binding protein 1"
}